{
  "gene_name": "Gremlin-2",
  "gene": "UniProtKB:Q9H772",
  "term_id": "GO:0038098",
  "gene_symbol": "GREM2",
  "term_label": "sequestering of BMP from receptor via BMP binding"
}